primary adaptive immune response [GO:0090720] (biological process) References: PMID:26831526 Sources: GOC:add Subtypes: primary adaptive immune response involving T cells and B cells [GO:0090721] Definition: An adaptive immune response against an antigen not previously encountered by immune system. Relationships: is a type of adaptive immune response [GO:0002250]